{
  "gene_name": "Immunoglobulin kappa variable 6D-21",
  "term_id": "GO:0006955",
  "term_label": "immune response",
  "gene": "UniProtKB:A0A0A0MT36",
  "gene_symbol": "IGKV6D-21"
}